{
  "gene_symbol": "GATA4",
  "gene": "UniProtKB:P43694",
  "term_id": "GO:0000122",
  "term_label": "negative regulation of transcription by RNA polymerase II",
  "gene_name": "Transcription factor GATA-4"
}